negative regulation of ribosomal protein gene transcription from RNA polymerase II promoter in response to chemical stimulus [GO:0010689] (biological process) Definition: Any process that decreases the frequency, rate or extent of the synthesis of RNA from ribosomal protein genes by RNA polymerase II, originating at an RNA polymerase II promoter, as a result of a chemical stimulus. Relationships: is a type of GO:0010688; is part of response to chemical [GO:0042221] Sources: GOC:dph, GOC:tb, GOC:txnOH